{
  "term_id": "GO:0005834",
  "gene_symbol": "GNAT1",
  "term_label": "heterotrimeric G-protein complex",
  "gene": "UniProtKB:P11488",
  "gene_name": "Guanine nucleotide-binding protein G(t) subunit alpha-1"
}